{
  "gene_name": "Ras association domain-containing protein 3",
  "gene": "UniProtKB:Q86WH2",
  "gene_symbol": "RASSF3",
  "term_id": "GO:0007165",
  "term_label": "signal transduction"
}